{
  "term_id": "GO:0015629",
  "gene": "UniProtKB:Q9NPC6",
  "term_label": "actin cytoskeleton",
  "gene_symbol": "MYOZ2",
  "gene_name": "Myozenin-2"
}